regulation of bleb assembly [GO:1904170] (biological process) Definition: Any process that modulates the frequency, rate or extent of bleb assembly. References: PMID:25651887 Sources: GOC:TermGenie, GOC:als, GO_REF:0000058 Also known as: regulation of cell blebbing Relationships: is a type of GO:0120032; RO_0002211 bleb assembly [GO:0032060] Subtypes: negative regulation of bleb assembly [GO:1904171], positive regulation of bleb assembly [GO:1904172]